{
  "gene_symbol": "OR2A14",
  "term_id": "GO:0005886",
  "gene_name": "Olfactory receptor 2A14",
  "term_label": "plasma membrane",
  "gene": "UniProtKB:Q96R47"
}